oxidoreductase activity, acting on other nitrogenous compounds as donors [GO:0016661] (molecular function) Sources: EC:1.7.-.- Definition: Catalysis of an oxidation-reduction (redox) reaction in which a nitrogenous group, excluding NH and NH2 groups, acts as a hydrogen or electron donor and reduces a hydrogen or electron acceptor. Relationships: is a type of oxidoreductase activity [GO:0016491] Also known as: oxidoreductase activity, acting on other nitrogenous compounds as donors, other acceptors Subtypes: nitrate reductase activity [GO:0008940], oxidoreductase activity, acting on other nitrogenous compounds as donors, cytochrome as acceptor [GO:0016662], GO:0016663, GO:0016664, oxidoreductase activity, acting on other nitrogenous compounds as donors, with NAD or NADP as acceptor [GO:0046857], hydroxylamine reductase activity [GO:0050418], nitrite reductase activity [GO:0098809]